glycine betaine-activated nonselective monoatomic cation channel activity [GO:0090686] (molecular function) References: PMID:24212673 Sources: GOC:kmv Definition: Enables the transmembrane transfer of a monoatomic cation by a channel that opens when glycine betaine has been bound by the channel complex or one of its constituent parts. Also known as: glycine betaine-activated nonselective monovalent cation channel activity Relationships: is a type of ligand-gated monoatomic cation channel activity [GO:0099094]